S-adenosylmethionine:tRNA ribosyltransferase-isomerase activity [GO:0051075] (molecular function) Also known as: S-adenosyl methionine:tRNA ribosyltransferase-isomerase activity Definition: Catalysis of the reaction: S-adenosylmethionine + 7-(aminomethyl)-7-deazaguanosine-tRNA = adenine + methionine + epoxyqueuosine-tRNA. 7-(aminomethyl)-7-deazaguanosine-tRNA is also known as preQ1-tRNA, and epoxyqueuosine-tRNA as oQ-tRNA. References: PMID:12731872 Relationships: is a type of glycosyltransferase activity [GO:0016757]; is a type of isomerase activity [GO:0016853]; is_a catalytic activity, acting on a tRNA [GO:0140101]